{
  "term_label": "cytoplasm",
  "gene": "UniProtKB:P55265",
  "gene_symbol": "ADAR",
  "term_id": "GO:0005737",
  "gene_name": "Double-stranded RNA-specific adenosine deaminase"
}